{
  "gene": "UniProtKB:P55773",
  "term_label": "cell chemotaxis",
  "term_id": "GO:0060326",
  "gene_symbol": "CCL23",
  "gene_name": "C-C motif chemokine 23"
}